{
  "gene_symbol": "FAXDC2",
  "gene": "UniProtKB:Q96IV6",
  "term_label": "endoplasmic reticulum membrane",
  "term_id": "GO:0005789",
  "gene_name": "Fatty acid hydroxylase domain-containing protein 2"
}